{
  "gene_name": "Amphiregulin",
  "term_label": "epidermal growth factor receptor signaling pathway",
  "term_id": "GO:0007173",
  "gene": "UniProtKB:P15514",
  "gene_symbol": "AREG"
}